phagocytosis [GO:0006909] (biological process) Definition: A vesicle-mediated transport process that results in the engulfment of external particulate material by phagocytes and their delivery to the lysosome. The particles are initially contained within phagocytic vacuoles (phagosomes), which then fuse with primary lysosomes to effect digestion of the particles. Subtypes: apoptotic cell clearance [GO:0043277] Sources: ISBN:0198506732 Relationships: is a type of endocytosis [GO:0006897] Regulation: regulated by regulation of phagocytosis [GO:0050764]; negatively regulated by negative regulation of phagocytosis [GO:0050765]; positively regulated by positive regulation of phagocytosis [GO:0050766]